{
  "gene_name": "Phosphatidylcholine:ceramide cholinephosphotransferase 1",
  "gene_symbol": "SGMS1",
  "gene": "UniProtKB:Q86VZ5",
  "term_label": "sphingomyelin synthase activity",
  "term_id": "GO:0033188"
}